crossed form four-way junction DNA binding [GO:0000402] (molecular function) Relationships: is a type of four-way junction DNA binding [GO:0000400] References: PMID:15563464 Sources: GOC:krc, ISBN:0815332181 Definition: Binding to a DNA segment containing the crossed form of a four-way junction, also known as a Holliday junction, a structure where two DNA double strands are held together by reciprocal exchange of two of the four strands, one strand each from the two original helices. The crossed form of a four-way junction cannot be diagrammed without any of the strands crossing over, and instead contains a single crossover between two of the strands. Also known as: crossed form Holliday junction binding